thioredoxin-disulfide reductase (NADPH) activity [GO:0004791] (molecular function) Sources: RHEA:20345 Relationships: is_a antioxidant activity [GO:0016209]; is a type of protein-disulfide reductase [NAD(P)H] activity [GO:0047134] Also known as: thioredoxin disulfide reductase activity, thioredoxin-disulfide reductase activity, thioredoxin-disulphide reductase activity, NADPH:oxidized thioredoxin oxidoreductase activity, thioredoxin reductase (NADPH) activity, thioredoxin-disulfide reductase (NADP) activity Definition: Catalysis of the reaction: thioredoxin-dithiol + NADP+ = thioredoxin-disulfide + H+ + NADPH.